{
  "gene_symbol": "TRIM31",
  "term_id": "GO:0005737",
  "gene": "UniProtKB:Q9BZY9",
  "term_label": "cytoplasm",
  "gene_name": "E3 ubiquitin-protein ligase TRIM31"
}